apoptotic process involved in metanephric collecting duct development [GO:1900204] (biological process) Relationships: is a type of apoptotic process involved in development [GO:1902742]; is part of metanephric collecting duct development [GO:0072205] Also known as: apoptotic cell death of metanephric collecting duct development, apoptotic process of metanephric collecting duct development, apoptotic programmed cell death of metanephric collecting duct development, programmed cell death by apoptosis of metanephric collecting duct development, apoptosis of metanephric collecting duct development, apoptotic program of metanephric collecting duct development, type I programmed cell death of metanephric collecting duct development, signaling (initiator) caspase activity of metanephric collecting duct development Regulation: RO_0002211 by GO:1900214; negatively regulated by negative regulation of apoptotic process involved in metanephric collecting duct development [GO:1900215]; positively regulated by positive regulation of apoptotic process involved in metanephric collecting duct development [GO:1900216] Definition: Any apoptotic process that is involved in metanephric collecting duct development. References: PMID:17314325 Sources: GOC:TermGenie, GOC:mtg_kidney_jan10, GOC:yaf